dCMP deaminase activity [GO:0004132] (MF) Definition: Catalysis of the reaction: dCMP + H2O = dUMP + NH3. Relationships: is a type of hydrolase activity, acting on carbon-nitrogen (but not peptide) bonds, in cyclic amidines [GO:0016814]; is a type of deaminase activity [GO:0019239] Also known as: dCMP aminohydrolase activity, deoxy-CMP-deaminase activity, deoxycytidine monophosphate deaminase activity, deoxycytidine-5'-monophosphate aminohydrolase activity, deoxycytidine-5'-phosphate deaminase activity, deoxycytidylate aminohydrolase activity, deoxycytidylate deaminase activity Sources: EC:3.5.4.12